{
  "term_label": "Unknown cellular component",
  "gene": "UniProtKB:Q5VV52",
  "term_id": "UNKNOWN:0003",
  "gene_name": "Zinc finger protein 691",
  "gene_symbol": "ZNF691"
}